{
  "term_label": "hydrolase activity",
  "gene_symbol": "HINT1",
  "gene": "UniProtKB:P49773",
  "gene_name": "Adenosine 5'-monophosphoramidase HINT1",
  "term_id": "GO:0016787"
}